{
  "term_id": "GO:0005525",
  "gene": "UniProtKB:Q8WXF7",
  "term_label": "GTP binding",
  "gene_symbol": "ATL1",
  "gene_name": "Atlastin-1"
}